{
  "term_id": "UNKNOWN:0001",
  "gene": "UniProtKB:P61962",
  "term_label": "Unknown molecular function",
  "gene_name": "DDB1- and CUL4-associated factor 7",
  "gene_symbol": "DCAF7"
}